{
  "gene": "UniProtKB:Q9Y4I1",
  "gene_symbol": "MYO5A",
  "term_id": "GO:0015629",
  "gene_name": "Unconventional myosin-Va",
  "term_label": "actin cytoskeleton"
}